{
  "gene_name": "5'-3' exonuclease PLD4",
  "gene": "UniProtKB:Q96BZ4",
  "gene_symbol": "PLD4",
  "term_label": "Unknown molecular function",
  "term_id": "UNKNOWN:0001"
}